{
  "gene": "UniProtKB:A8MT66",
  "gene_name": "Putative uncharacterized protein ENSP00000383407",
  "gene_symbol": "A8MT66",
  "term_label": "Unknown cellular component",
  "term_id": "UNKNOWN:0003"
}